{
  "gene_name": "Kelch-like protein 2",
  "term_label": "cytoplasm",
  "gene": "UniProtKB:O95198",
  "term_id": "GO:0005737",
  "gene_symbol": "KLHL2"
}